{
  "term_label": "negative regulation of translation",
  "gene_symbol": "CNOT10",
  "gene": "UniProtKB:Q9H9A5",
  "gene_name": "CCR4-NOT transcription complex subunit 10",
  "term_id": "GO:0017148"
}